{
  "gene": "UniProtKB:Q6PK18",
  "gene_name": "2-oxoglutarate and iron-dependent oxygenase domain-containing protein 3",
  "term_label": "Unknown molecular function",
  "gene_symbol": "OGFOD3",
  "term_id": "UNKNOWN:0001"
}